{
  "gene_symbol": "GUCA2A",
  "gene_name": "Guanylin",
  "term_label": "Unknown cellular component",
  "term_id": "UNKNOWN:0003",
  "gene": "UniProtKB:Q02747"
}